{
  "gene_symbol": "OR14A16",
  "gene_name": "Olfactory receptor 14A16",
  "gene": "UniProtKB:Q8NHC5",
  "term_label": "Unknown cellular component",
  "term_id": "UNKNOWN:0003"
}